glucosinolate biosynthetic process from phenylalanine [GO:0033507] (biological process) Sources: GOC:mah, MetaCyc:PWY-2821 Also known as: glucosinolate anabolism from phenylalanine, glucosinolate biosynthesis from phenylalanine, glucosinolate formation from phenylalanine, glucosinolate synthesis from phenylalanine Definition: The chemical reactions and pathways resulting in the formation of glucosinolates from other compounds including phenylalanine. Relationships: is a type of carboxylic acid metabolic process [GO:0019752]; is a type of glucosinolate biosynthetic process [GO:0019761]